{
  "term_label": "Unknown cellular component",
  "term_id": "UNKNOWN:0003",
  "gene_name": "Dendrin",
  "gene_symbol": "DDN",
  "gene": "UniProtKB:O94850"
}